{
  "term_id": "GO:0006357",
  "term_label": "regulation of transcription by RNA polymerase II",
  "gene_symbol": "MLXIPL",
  "gene": "UniProtKB:Q9NP71",
  "gene_name": "Carbohydrate-responsive element-binding protein"
}